{
  "gene": "UniProtKB:Q8N8V8",
  "term_label": "Unknown cellular component",
  "gene_symbol": "TMEM105",
  "gene_name": "Transmembrane protein 105",
  "term_id": "UNKNOWN:0003"
}